{
  "gene_symbol": "TUBB6",
  "term_label": "mitotic cell cycle",
  "term_id": "GO:0000278",
  "gene_name": "Tubulin beta-6 chain",
  "gene": "UniProtKB:Q9BUF5"
}